sterol 14-demethylase activity [GO:0008398] (molecular function) Relationships: is a type of oxidoreductase activity, acting on paired donors, with incorporation or reduction of molecular oxygen, NAD(P)H as one donor, and incorporation of one atom of oxygen [GO:0016709]; is a type of demethylase activity [GO:0032451] Also known as: cytochrome P450 51 activity, cytochrome P450 CYP51, lanosterol 14-alpha-demethylase activity, lanosterol 14-demethylase activity, obtusufoliol 14-demethylase activity, lanosterol 14alpha-demethylase activity, sterol 14-alpha-demethylase activity, sterol 14alpha-demethylase activity Definition: Catalysis of the reaction: a 14alpha-methyl steroid + 3 O2 + 3 reduced [NADPH-hemoprotein reductase] = a delta14 steroid + formate + 4 H+ + 4 H2O + 3 oxidized [NADPH-hemoprotein reductase]. Sources: RHEA:54028